{
  "term_label": "Toll signaling pathway",
  "term_id": "GO:0008063",
  "gene": "UniProtKB:P51617",
  "gene_name": "Interleukin-1 receptor-associated kinase 1",
  "gene_symbol": "IRAK1"
}